{
  "term_id": "UNKNOWN:0003",
  "gene": "UniProtKB:Q8WVI0",
  "gene_name": "Ubiquinol-cytochrome-c reductase complex assembly factor 5",
  "term_label": "Unknown cellular component",
  "gene_symbol": "UQCC5"
}